{
  "term_id": "UNKNOWN:0003",
  "gene_symbol": "PPP1R18",
  "term_label": "Unknown cellular component",
  "gene": "UniProtKB:Q6NYC8",
  "gene_name": "Phostensin"
}